inositol phosphorylceramide phospholipase activity [GO:0052713] (molecular function) Sources: GOC:ai Relationships: is a type of inositol phosphosphingolipid phospholipase activity [GO:0052712] Subtypes: mannosyl-inositol phosphorylceramide phospholipase activity [GO:0052714], GO:0052715 Definition: Catalysis of the reaction: inositol phosphorylceramide + H2O = C26-phytoceramide + phosphorylinositol.